{
  "term_label": "alcohol dehydrogenase (NADP+) activity",
  "gene_name": "Voltage-gated potassium channel subunit beta-1",
  "gene": "UniProtKB:Q14722",
  "term_id": "GO:0008106",
  "gene_symbol": "KCNAB1"
}